{
  "gene": "UniProtKB:Q9H9V9",
  "gene_symbol": "JMJD4",
  "term_label": "positive regulation of translational termination",
  "gene_name": "2-oxoglutarate and iron-dependent oxygenase JMJD4",
  "term_id": "GO:0045905"
}